{
  "gene_name": "Zinc finger matrin-type protein 5",
  "term_id": "UNKNOWN:0001",
  "gene": "UniProtKB:Q9UDW3",
  "gene_symbol": "ZMAT5",
  "term_label": "Unknown molecular function"
}